{
  "term_id": "GO:0019731",
  "gene_name": "Defensin-6",
  "gene_symbol": "DEFA6",
  "term_label": "antibacterial humoral response",
  "gene": "UniProtKB:Q01524"
}